{
  "gene": "UniProtKB:Q92902",
  "gene_name": "BLOC-3 complex member HPS1",
  "gene_symbol": "HPS1",
  "term_label": "melanosome assembly",
  "term_id": "GO:1903232"
}